{
  "term_label": "protein serine/threonine kinase activity",
  "gene_name": "Dual specificity tyrosine-phosphorylation-regulated kinase 1B",
  "term_id": "GO:0004674",
  "gene_symbol": "DYRK1B",
  "gene": "UniProtKB:Q9Y463"
}